{
  "gene": "UniProtKB:Q9GIP4",
  "gene_name": "Putative L-type amino acid transporter 1-like protein IMAA",
  "term_id": "UNKNOWN:0002",
  "term_label": "Unknown biological process",
  "gene_symbol": "SLC7A5P2"
}